clathrin coat [GO:0030118] (cellular component) Definition: A membrane coat found on coated pits and some coated vesicles; consists of polymerized clathrin triskelions, each comprising three clathrin heavy chains and three clathrin light chains, linked to the membrane via one of the AP adaptor complexes. Subtypes: GO:0030125, GO:0030132 References: PMID:11252894, PMID:9531549 Sources: GOC:mah Also known as: clathrin cage Relationships: is a type of GO:0030117